regulation of metaxylem development [GO:0090060] (biological process) Definition: Any process that modulates the frequency, rate, or extent of metaxylem development. Metaxylem development is the process whose specific outcome is the progression of the metaxylem over time, from its formation to the mature structure. The metaxylem is the part of the primary xylem that differentiates after the protoxylem and before the secondary xylem, if any of the latter is formed. Relationships: is a type of regulation of multicellular organismal development [GO:2000026]; regulates metaxylem development [GO:0090058] Sources: GOC:dph, GOC:sdb_2009, GOC:tb